L-isoleucine-2-oxoglutarate transaminase activity [GO:0052656] (molecular function) Sources: RHEA:24801 Relationships: is a type of GO:0004084 Definition: Catalysis of the reaction: 2-oxoglutarate + L-isoleucine = (S)-3-methyl-2-oxopentanoic acid + L-glutamic acid. Also known as: L-isoleucine aminotransferase activity